conus arteriosus formation [GO:0003240] (biological process) Relationships: is a type of GO:0003207; is part of conus arteriosus morphogenesis [GO:0003239] Definition: The developmental process pertaining to the initial formation of the conus arteriosus from unspecified parts. The conus arteriosus is a valved chamber with thick muscular walls stemming from the ventricle and connecting to the pulmonary trunk. Sources: GOC:mtg_heart